{
  "term_id": "GO:0036376",
  "gene_name": "Potassium-transporting ATPase alpha chain 1",
  "gene": "UniProtKB:P20648",
  "gene_symbol": "ATP4A",
  "term_label": "sodium ion export across plasma membrane"
}